{
  "term_label": "regulation of transcription by RNA polymerase II",
  "gene_name": "Double homeobox protein 4-like protein 2",
  "gene": "UniProtKB:P0CJ85",
  "gene_symbol": "DUX4L2",
  "term_id": "GO:0006357"
}